{
  "gene_symbol": "HDAC9",
  "gene": "UniProtKB:Q9UKV0",
  "term_label": "histone deacetylase complex",
  "term_id": "GO:0000118",
  "gene_name": "Histone deacetylase 9"
}